{
  "term_label": "Unknown molecular function",
  "gene_symbol": "CASKIN2",
  "gene": "UniProtKB:Q8WXE0",
  "gene_name": "Caskin-2",
  "term_id": "UNKNOWN:0001"
}